{
  "gene_symbol": "H2BC12",
  "gene": "UniProtKB:O60814",
  "gene_name": "Histone H2B type 1-K",
  "term_id": "GO:0030527",
  "term_label": "structural constituent of chromatin"
}